positive regulation of potassium ion transport [GO:0043268] (biological process) Sources: GOC:jl Also known as: positive regulation of K+ transport, positive regulation of potassium transport, up regulation of potassium ion transport, up-regulation of potassium ion transport, upregulation of potassium ion transport, activation of potassium ion transport, positive regulation of K+ conductance, positive regulation of potassium conductance, positive regulation of potassium ion conductance, stimulation of potassium ion transport Subtypes: positive regulation of potassium ion transmembrane transport [GO:1901381] Relationships: is a type of regulation of potassium ion transport [GO:0043266]; is a type of positive regulation of monoatomic ion transport [GO:0043270]; positively regulates GO:0006813 Definition: Any process that activates or increases the frequency, rate or extent of the directed movement of potassium ions (K+) into, out of or within a cell, or between cells, by means of some agent such as a transporter or pore.